{
  "term_id": "UNKNOWN:0003",
  "gene": "UniProtKB:Q13630",
  "gene_name": "GDP-L-fucose synthase",
  "gene_symbol": "GFUS",
  "term_label": "Unknown cellular component"
}